{
  "gene_name": "Septin-1",
  "term_id": "GO:0031105",
  "gene": "UniProtKB:Q8WYJ6",
  "gene_symbol": "SEPTIN1",
  "term_label": "septin complex"
}